negative regulation of neural crest cell differentiation [GO:1905293] (BP) Subtypes: GO:1905296 Definition: Any process that stops, prevents or reduces the frequency, rate or extent of neural crest cell differentiation. Relationships: is a type of negative regulation of multicellular organismal process [GO:0051241]; is a type of regulation of neural crest cell differentiation [GO:1905292]; is a type of negative regulation of stem cell differentiation [GO:2000737]; negatively regulates GO:0014033 References: PMID:15073157 Sources: GOC:BHF, GOC:TermGenie, GOC:rl, GO_REF:0000058 Also known as: down regulation of neural crest cell differentiation, down-regulation of neural crest cell differentiation, downregulation of neural crest cell differentiation, inhibition of neural crest cell differentiation